lycopene epsilon cyclase activity [GO:0045435] (molecular function) Also known as: lycopene cyclase Relationships: is a type of cyclase activity [GO:0009975]; is a type of intramolecular oxidoreductase activity [GO:0016860] Definition: Catalysis of the cyclization of an epsilon ring at one end of the lycopene molecule (psi, psi-carotene) to form delta-carotene (epsilon, psi-carotene). References: PMID:8837512